{
  "gene_name": "GTPase-activating Rap_Ran-GAP domain-like protein 3",
  "term_label": "GTPase activator activity",
  "term_id": "GO:0005096",
  "gene_symbol": "GARNL3",
  "gene": "UniProtKB:Q5VVW2"
}